N-hydroxy-2-acetamidofluorene reductase [NAD(P)H] activity [GO:0047137] (molecular function) Sources: EC:1.7.1.12 Definition: Catalysis of the reaction: 2-acetamidofluorene + NAD(P)+ + H2O = N-hydroxy-2-acetamidofluorene + NAD(P)H + H+. Relationships: is a type of GO:0046857 Also known as: 2-acetamidofluorene:NAD(P)+ oxidoreductase activity, N-hydroxy-2-acetylaminofluorene reductase activity, NAD(P)H2:N-hydroxy-2-acetamidofluorene N-oxidoreductase activity, NAD(P)H:N-hydroxy-2-acetamidofluorene N-oxidoreductase activity